{
  "gene_name": "Coiled-coil domain-containing protein 68",
  "term_id": "UNKNOWN:0001",
  "gene": "UniProtKB:Q9H2F9",
  "term_label": "Unknown molecular function",
  "gene_symbol": "CCDC68"
}